{
  "gene": "UniProtKB:A6NNW6",
  "gene_name": "Enolase 4",
  "term_id": "GO:0000015",
  "gene_symbol": "ENO4",
  "term_label": "phosphopyruvate hydratase complex"
}